regulation of stomatal movement [GO:0010119] (biological process) Subtypes: GO:0090333, regulation of stomatal opening [GO:1902456] Relationships: is a type of regulation of cellular process [GO:0050794]; regulates stomatal movement [GO:0010118] Definition: Any process that modulates the frequency, rate or extent of stomatal movement. Sources: GOC:sm